{
  "gene_symbol": "CBFB",
  "gene_name": "Core-binding factor subunit beta",
  "term_label": "core-binding factor complex",
  "gene": "UniProtKB:Q13951",
  "term_id": "GO:0016513"
}